{
  "gene": "UniProtKB:O75317",
  "term_id": "GO:0031647",
  "gene_symbol": "USP12",
  "term_label": "regulation of protein stability",
  "gene_name": "Ubiquitin carboxyl-terminal hydrolase 12"
}